2-(hydroxymethyl)-3-(acetamidomethylene)succinate hydrolase activity [GO:0047414] (molecular function) Definition: Catalysis of the reaction: (2Z)-2-(acetamidomethylene)-3-(hydroxymethyl)succinate + 2 H2O + H+ = 2-(hydroxymethyl)-4-oxobutanoate + acetate + CO2 + NH4. Relationships: is a type of hydrolase activity, acting on carbon-nitrogen (but not peptide) bonds, in linear amides [GO:0016811] Also known as: 2-(hydroxymethyl)-3-(acetamidomethylene)succinate amidohydrolase (deaminating, decarboxylating), alpha-hydroxymethyl-alpha'-(N-acetylaminomethylene)succinic acid hydrolase activity, compound B hydrolase activity Sources: EC:3.5.1.66, RHEA:17677